{
  "term_label": "immune response",
  "term_id": "GO:0006955",
  "gene_name": "Immunoglobulin lambda variable 1-51",
  "gene_symbol": "IGLV1-51",
  "gene": "UniProtKB:P01701"
}